{
  "gene": "UniProtKB:P48736",
  "gene_symbol": "PIK3CG",
  "term_id": "GO:0016303",
  "term_label": "1-phosphatidylinositol-3-kinase activity",
  "gene_name": "Phosphatidylinositol 4,5-bisphosphate 3-kinase catalytic subunit gamma isoform"
}